{
  "gene_symbol": "ARF3",
  "term_id": "GO:0005737",
  "gene": "UniProtKB:P61204",
  "gene_name": "ADP-ribosylation factor 3",
  "term_label": "cytoplasm"
}